{
  "gene_symbol": "SLFN5",
  "term_id": "UNKNOWN:0001",
  "gene_name": "Schlafen family member 5",
  "gene": "UniProtKB:Q08AF3",
  "term_label": "Unknown molecular function"
}